response to N-phenylthiourea [GO:1902610] (biological process) References: PMID:24006265 Sources: GOC:TermGenie, GOC:rjd, GO_REF:0000071 Relationships: is a type of GO:0042221 Subtypes: cellular response to N-phenylthiourea [GO:1902611] Definition: Any process that results in a change in state or activity of a cell or an organism (in terms of movement, secretion, enzyme production, gene expression, etc.) as a result of a N-phenylthiourea stimulus.